{
  "gene_name": "GDNF family receptor alpha-2",
  "gene_symbol": "GFRA2",
  "gene": "UniProtKB:O00451",
  "term_id": "GO:0007399",
  "term_label": "nervous system development"
}